regulation of branching involved in salivary gland morphogenesis by epithelial-mesenchymal signaling [GO:0060683] (biological process) References: PMID:18559345 Sources: GOC:dph Also known as: regulation of branching involved in salivary gland morphogenesis by epithelial-mesenchymal signalling Relationships: is a type of epithelial-mesenchymal cell signaling [GO:0060684]; is a type of regulation of branching involved in salivary gland morphogenesis [GO:0060693] Definition: Any process that modulates the rate, frequency, or extent of salivary gland branching as a result of the transfer of information from the epithelial cells to the mesenchymal cells of the salivary gland.